RNA-3'-phosphate cyclase activity [GO:0003963] (molecular function) Relationships: is a type of cyclase activity [GO:0009975]; is a type of ligase activity, forming phosphoric ester bonds [GO:0016886]; is a type of catalytic activity, acting on RNA [GO:0140098] Definition: Catalysis of the reaction: ATP + RNA 3'-terminal-phosphate = AMP + diphosphate + RNA terminal-2',3'-cyclic-phosphate. Also known as: RNA 3'-terminal phosphate cyclase activity, RNA cyclase activity, RNA-3'-phosphate:RNA ligase (cyclizing, AMP-forming) Sources: EC:6.5.1.4